acyl-CoA 11-(Z)-desaturase activity [GO:0017105] (MF) Also known as: Z/E11-desaturase, acyl-CoA delta11-desaturase activity, delta(11) desaturase, delta(11)-fatty-acid desaturase, fatty acid delta(11)-desaturase, acyl-CoA D11-desaturase activity, acyl-CoA delta(11)-desaturase activity, acyl-CoA delta11-(Z)-desaturase activity, delta(11)-palmitoyl-CoA desaturase, myristoyl-CoA 11-(Z) desaturase activity References: PMID:15063718, PMID:15544945 Sources: RHEA:25852 Definition: Catalysis of the reaction: an 11,12-saturated fatty acyl-CoA + 2 Fe(II)-[cytochrome b5] + 2 H+ + O2 = an (11Z)-delta-11-fatty acyl-CoA + 2 Fe(III)-[cytochrome b5] + 2 H2O. Relationships: is a type of acyl-CoA desaturase activity [GO:0016215]